{
  "gene_name": "Transcriptional coactivator YAP1",
  "term_label": "transcription corepressor activity",
  "gene": "UniProtKB:P46937",
  "gene_symbol": "YAP1",
  "term_id": "GO:0003714"
}